{
  "gene_name": "UDP-glucuronosyltransferase 1A7",
  "gene": "UniProtKB:Q9HAW7",
  "term_id": "GO:0051552",
  "term_label": "flavone metabolic process",
  "gene_symbol": "UGT1A7"
}